{
  "term_id": "GO:0010664",
  "gene_symbol": "BAG3",
  "gene_name": "BAG family molecular chaperone regulator 3",
  "gene": "UniProtKB:O95817",
  "term_label": "negative regulation of striated muscle cell apoptotic process"
}